{
  "term_id": "GO:0005634",
  "term_label": "nucleus",
  "gene_name": "Poly(rC)-binding protein 4",
  "gene": "UniProtKB:P57723",
  "gene_symbol": "PCBP4"
}